{
  "term_id": "GO:0006406",
  "gene_name": "Nuclear pore complex protein Nup85",
  "gene": "UniProtKB:Q9BW27",
  "gene_symbol": "NUP85",
  "term_label": "mRNA export from nucleus"
}